glucose catabolic process to lactate [GO:0019659] (biological process) Definition: The anaerobic enzymatic chemical reactions and pathways resulting in the breakdown of glucose to lactate, and possibly ethanol, yielding energy in the form of adenosine triphosphate (ATP). Also known as: glucose fermentation to lactate, lactate fermentation Relationships: is a type of GO:0006007; is a type of lactate metabolic process [GO:0006089]; is a type of GO:0006113 Subtypes: glucose catabolic process to D-lactate and ethanol [GO:0019656], glucose fermentation to lactate and acetate [GO:0019658], glucose catabolic process to lactate via pyruvate [GO:0019661] Sources: GOC:jl